{
  "gene_symbol": "ZNF222",
  "gene_name": "Zinc finger protein 222",
  "term_id": "UNKNOWN:0003",
  "gene": "UniProtKB:Q9UK12",
  "term_label": "Unknown cellular component"
}